{
  "term_id": "UNKNOWN:0003",
  "gene_name": "O-phosphoseryl-tRNA(Sec) selenium transferase",
  "gene_symbol": "SEPSECS",
  "gene": "UniProtKB:Q9HD40",
  "term_label": "Unknown cellular component"
}